positive regulation of trophoblast cell migration [GO:1901165] (biological process) Sources: GOC:BHF, GOC:TermGenie Relationships: is_a GO:0030335; is a type of GO:0051094; is a type of positive regulation of multicellular organismal process [GO:0051240]; is a type of regulation of trophoblast cell migration [GO:1901163]; is a type of positive regulation of reproductive process [GO:2000243]; RO_0002213 trophoblast cell migration [GO:0061450] Also known as: up regulation of trophoblast cell migration, up-regulation of trophoblast cell migration, upregulation of trophoblast cell migration, activation of trophoblast cell migration Definition: Any process that activates or increases the frequency, rate or extent of trophoblast cell migration.